T cell cytokine production [GO:0002369] (biological process) Regulation: regulated by GO:0002724; negatively regulated by GO:0002725; positively regulated by positive regulation of T cell cytokine production [GO:0002726] Relationships: is a type of cytokine production involved in immune response [GO:0002367]; is a type of T cell mediated immunity [GO:0002456] Subtypes: CD4-positive, alpha-beta T cell cytokine production [GO:0035743] Definition: Any process that contributes to cytokine production by a T cell. Also known as: T lymphocyte cytokine production, T-cell cytokine production, T-lymphocyte cytokine production Sources: GOC:add, ISBN:0781735149 Note: Note that this term is in the subset of terms that should not be used for direct gene product annotation. Instead, select one of the 'regulation' children terms.